{
  "gene": "UniProtKB:Q8NH10",
  "gene_name": "Olfactory receptor 8U1",
  "term_id": "UNKNOWN:0003",
  "term_label": "Unknown cellular component",
  "gene_symbol": "OR8U1"
}